{
  "gene_name": "AP-3 complex subunit beta-1",
  "term_label": "Unknown molecular function",
  "gene": "UniProtKB:O00203",
  "term_id": "UNKNOWN:0001",
  "gene_symbol": "AP3B1"
}